symbiont-mediated perturbation of host actin cytoskeleton via actin polymerization [GO:0141033] (biological process) Definition: The process in which an organism effects a change that impairs the structure or function of the host actin cytoskeleton by polymerizing the host filamentous actin. The host is defined as the larger of the organisms involved in a symbiotic interaction. References: PMID:18331467, PMID:25293534 Also known as: perturbation by symbiont of host actin cytoskeleton via actin polymerization Relationships: is a type of symbiont-mediated perturbation of host actin cytoskeleton [GO:0141027]